{
  "term_id": "GO:0005783",
  "gene_name": "Alpha-1,3-mannosyl-glycoprotein 4-beta-N-acetylglucosaminyltransferase A",
  "gene_symbol": "MGAT4A",
  "term_label": "endoplasmic reticulum",
  "gene": "UniProtKB:Q9UM21"
}